{
  "term_id": "GO:0048240",
  "term_label": "sperm capacitation",
  "gene": "UniProtKB:Q9HAT0",
  "gene_symbol": "ROPN1",
  "gene_name": "Ropporin-1A"
}